{
  "term_label": "protein-containing complex",
  "gene_name": "Protein-lysine N-methyltransferase EEF2KMT",
  "gene_symbol": "EEF2KMT",
  "term_id": "GO:0032991",
  "gene": "UniProtKB:Q96G04"
}